{
  "gene": "UniProtKB:O95196",
  "term_label": "axon regeneration",
  "gene_name": "Chondroitin sulfate proteoglycan 5",
  "gene_symbol": "CSPG5",
  "term_id": "GO:0031103"
}